disaccharide binding [GO:0048030] (molecular function) Subtypes: lactose binding [GO:0030395], cellobiose binding [GO:0044585], maltose binding [GO:1901982], melibiose binding [GO:1903777] Sources: GOC:jid Relationships: is a type of GO:0070492 Definition: Binding to a disaccharide. Disaccharides are sugars composed of two monosaccharide units.